{
  "gene_name": "Serine_arginine-rich splicing factor 1",
  "term_label": "nuclear speck",
  "gene_symbol": "SRSF1",
  "term_id": "GO:0016607",
  "gene": "UniProtKB:Q07955"
}